{
  "gene": "UniProtKB:Q13393",
  "gene_name": "Phospholipase D1",
  "term_label": "phospholipase D activity",
  "term_id": "GO:0004630",
  "gene_symbol": "PLD1"
}